neutrophil homeostasis [GO:0001780] (biological process) References: PMID:12752675, PMID:12960266 Sources: GOC:add, GOC:pr Note: Note that this term represents the return of neutrophil levels to stable numbers following an immune response as well as the proliferation and elimination of neutrophils required to maintain stable numbers in the absence of an outside stimulus. Definition: The process of regulating the proliferation and elimination of neutrophils such that the total number of neutrophils within a whole or part of an organism is stable over time in the absence of an outside stimulus. Relationships: is a type of leukocyte homeostasis [GO:0001776]; is a type of myeloid cell homeostasis [GO:0002262]